Lsd1/2 complex [GO:0033193] (cellular component) Relationships: is a type of protein-containing complex [GO:0032991]; is part of GO:0005694 Definition: A nucleosome-binding protein complex that comprises two SWIRM domain histone demethylases and two PHD finger proteins. The complex is involved in transcriptional regulation via heterochromatic silencing and the regulation of chromatin boundary formation, and was first identified in fission yeast. References: PMID:17371846, PMID:17434129, PMID:17440621 Sources: GOC:vw Also known as: SAPHIRE complex, Swm complex, Swm1/2 complex